{
  "gene_name": "Tektin-3",
  "term_id": "GO:0036126",
  "term_label": "sperm flagellum",
  "gene_symbol": "TEKT3",
  "gene": "UniProtKB:Q9BXF9"
}